{
  "gene_symbol": "H2AC12",
  "term_id": "GO:0031507",
  "term_label": "heterochromatin formation",
  "gene_name": "Histone H2A type 1-H",
  "gene": "UniProtKB:Q96KK5"
}